{
  "term_label": "cytoplasm",
  "term_id": "GO:0005737",
  "gene_symbol": "ATP5IF1",
  "gene_name": "ATPase inhibitor, mitochondrial",
  "gene": "UniProtKB:Q9UII2"
}